{
  "term_label": "transforming growth factor beta receptor signaling pathway",
  "gene": "UniProtKB:Q99717",
  "gene_symbol": "SMAD5",
  "gene_name": "Mothers against decapentaplegic homolog 5",
  "term_id": "GO:0007179"
}